gap junction channel activity involved in atrial cardiac muscle cell-AV node cell electrical coupling [GO:0086076] (molecular function) Also known as: gap junction channel activity involved in atrial cardiomyocyte-atrioventricular node cell electrical coupling, gap junction channel activity involved in atrial cardiomyocyte-AV node cell electrical coupling Relationships: is a type of GO:0086075; is part of atrial cardiac muscle cell to AV node cell communication by electrical coupling [GO:0086044] Sources: GOC:BHF, GOC:mtg_cardiac_conduct_nov11 Definition: A wide pore channel activity that enables a direct cytoplasmic connection from an atrial cardiomyocyte to an AV node cell. The gap junction passes electrical signals between the cells contributing to cardiac conduction.